glycolipid catabolic process [GO:0019377] (biological process) Sources: GOC:go_curators Definition: The chemical reactions and pathways resulting in the breakdown of glycolipid, a class of 1,2-di-O-acylglycerols joined at oxygen 3 by a glycosidic linkage to a carbohydrate part (usually a mono-, di- or tri-saccharide). Also known as: glycolipid breakdown, glycolipid catabolism, glycolipid degradation Relationships: is a type of glycolipid metabolic process [GO:0006664]; is a type of membrane lipid catabolic process [GO:0046466]; is a type of carbohydrate derivative catabolic process [GO:1901136] Subtypes: galactolipid catabolic process [GO:0019376], sophorosyloxydocosanoate catabolic process [GO:0019436], GO:0046479